{
  "gene_symbol": "PDE7B",
  "term_label": "3',5'-cyclic-AMP phosphodiesterase activity",
  "term_id": "GO:0004115",
  "gene_name": "cAMP-specific 3',5'-cyclic phosphodiesterase 7B",
  "gene": "UniProtKB:Q9NP56"
}